{
  "gene_name": "Ras-related protein Rab-5B",
  "term_id": "GO:0006897",
  "term_label": "endocytosis",
  "gene_symbol": "RAB5B",
  "gene": "UniProtKB:P61020"
}